{
  "term_label": "NADH dehydrogenase activity",
  "gene": "UniProtKB:P03905",
  "term_id": "GO:0003954",
  "gene_symbol": "MT-ND4",
  "gene_name": "NADH-ubiquinone oxidoreductase chain 4"
}